{
  "gene_symbol": "DTWD1",
  "gene": "UniProtKB:Q8N5C7",
  "term_label": "nucleus",
  "gene_name": "tRNA-uridine aminocarboxypropyltransferase 1",
  "term_id": "GO:0005634"
}